sporocarp development involved in asexual reproduction [GO:0000905] (biological process) Definition: The formation of a spore-bearing structure by fungus where spores will arise from asexual reproduction. Relationships: is a type of GO:0030584; is part of asexual reproduction [GO:0019954] Sources: GOC:clt, GOC:mtg_sensu Also known as: fruiting body formation involved in asexual reproduction, conidium development, imperfect stage fruiting body development, haploid fruiting, homokaryotic fruiting, monokaryotic fruiting